{
  "gene": "UniProtKB:Q8TBH0",
  "term_id": "GO:0005737",
  "term_label": "cytoplasm",
  "gene_symbol": "ARRDC2",
  "gene_name": "Arrestin domain-containing protein 2"
}